{
  "gene_name": "Long-chain fatty acid transport protein 2",
  "term_label": "long-chain fatty acid import into cell",
  "gene_symbol": "SLC27A2",
  "gene": "UniProtKB:O14975",
  "term_id": "GO:0044539"
}